{
  "term_id": "GO:0050911",
  "gene": "UniProtKB:Q8NGE3",
  "gene_symbol": "OR10P1",
  "term_label": "detection of chemical stimulus involved in sensory perception of smell",
  "gene_name": "Olfactory receptor 10P1"
}